{
  "gene": "UniProtKB:Q15738",
  "term_id": "GO:0008203",
  "term_label": "cholesterol metabolic process",
  "gene_name": "Sterol-4-alpha-carboxylate 3-dehydrogenase, decarboxylating",
  "gene_symbol": "NSDHL"
}